{
  "term_label": "B cell differentiation",
  "gene_name": "B-cell antigen receptor complex-associated protein beta chain",
  "gene_symbol": "CD79B",
  "term_id": "GO:0030183",
  "gene": "UniProtKB:P40259"
}